{
  "term_id": "GO:0005737",
  "gene_name": "Rho guanine nucleotide exchange factor 1",
  "term_label": "cytoplasm",
  "gene": "UniProtKB:Q92888",
  "gene_symbol": "ARHGEF1"
}